{
  "gene_name": "Serine_threonine-protein kinase PAK 5",
  "gene": "UniProtKB:Q9P286",
  "gene_symbol": "PAK5",
  "term_id": "GO:0004674",
  "term_label": "protein serine/threonine kinase activity"
}